{
  "term_label": "SWI/SNF complex",
  "gene_symbol": "SMARCD1",
  "gene_name": "SWI_SNF-related matrix-associated actin-dependent regulator of chromatin subfamily D member 1",
  "gene": "UniProtKB:Q96GM5",
  "term_id": "GO:0016514"
}